histone H4K20 demethylase activity [GO:0035575] (molecular function) Relationships: is a type of 2-oxoglutarate-dependent dioxygenase activity [GO:0016706]; is a type of histone H4 demethylase activity [GO:0141058] References: PMID:20622853, PMID:26214369, PMID:32209475 Also known as: histone H4-K20 demethylase activity, histone H4-methyl-lysine-20 demethylase activity, histone H4K20me demethylase activity, histone demethylase activity (H4-K20 specific), histone demethylase activity (H4K20-specific) Note: Note that the residue position corresponds to the canonical human H4 histone (UniProtKB:P02309); this residue is conserved across all eukaryotes. Note that the initiation methionine is cleaved, so the first residue is S1. Definition: Catalysis of the removal of the methyl group from a modified lysine residue at position 20 of the histone H4 protein. This is a dioxygenase reaction that is dependent on Fe(II) and 2-oxoglutarate.